{
  "gene_symbol": "NECTIN4",
  "term_label": "cell adhesion mediator activity",
  "gene_name": "Nectin-4",
  "term_id": "GO:0098631",
  "gene": "UniProtKB:Q96NY8"
}